{
  "gene_name": "Cadherin-24",
  "term_label": "adherens junction",
  "term_id": "GO:0005912",
  "gene": "UniProtKB:Q86UP0",
  "gene_symbol": "CDH24"
}